{
  "gene": "UniProtKB:P06727",
  "gene_name": "Apolipoprotein A-IV",
  "term_id": "GO:1903561",
  "gene_symbol": "APOA4",
  "term_label": "extracellular vesicle"
}